{
  "gene": "UniProtKB:P50458",
  "term_label": "neuron differentiation",
  "gene_name": "LIM_homeobox protein Lhx2",
  "term_id": "GO:0030182",
  "gene_symbol": "LHX2"
}